{
  "term_label": "nucleus",
  "gene": "UniProtKB:O43186",
  "gene_symbol": "CRX",
  "gene_name": "Cone-rod homeobox protein",
  "term_id": "GO:0005634"
}